fibroblast growth factor receptor signaling pathway involved in negative regulation of apoptotic process in bone marrow cell [GO:0035602] (biological process) Also known as: FGF receptor signaling pathway involved in negative regulation of apoptosis in bone marrow, FGFR signaling pathway involved in negative regulation of apoptosis in bone marrow, fibroblast growth factor receptor signaling pathway involved in negative regulation of apoptotic process in bone marrow, fibroblast growth factor receptor signalling pathway involved in negative regulation of apoptotic process in bone marrow, fibroblast growth factor receptor signaling pathway involved in negative regulation of apoptosis in bone marrow Relationships: is a type of GO:0008543; is part of negative regulation of apoptotic process in bone marrow cell [GO:0071866] Sources: GOC:mtg_apoptosis, GOC:yaf Definition: The series of molecular signals generated as a consequence of a fibroblast growth factor receptor binding to one of its physiological ligands, which stops, prevents, or reduces the frequency, rate or extent of the occurrence or rate of cell death by apoptotic process in the bone marrow.